{
  "gene": "UniProtKB:A6NCJ1",
  "gene_symbol": "TEKTIP1",
  "gene_name": "Tektin bundle-interacting protein 1",
  "term_label": "axonemal A tubule inner sheath",
  "term_id": "GO:0160111"
}